{
  "term_id": "UNKNOWN:0003",
  "gene_name": "POU domain, class 5, transcription factor 2",
  "gene_symbol": "POU5F2",
  "gene": "UniProtKB:Q8N7G0",
  "term_label": "Unknown cellular component"
}